{
  "term_id": "GO:0032956",
  "term_label": "regulation of actin cytoskeleton organization",
  "gene_symbol": "ARAP1",
  "gene_name": "Arf-GAP with Rho-GAP domain, ANK repeat and PH domain-containing protein 1",
  "gene": "UniProtKB:Q96P48"
}